positive regulation of snRNA pseudouridine synthesis [GO:1905358] (biological process) Also known as: up regulation of snRNA pseudouridine synthesis, up-regulation of snRNA pseudouridine synthesis, upregulation of snRNA pseudouridine synthesis, activation of snRNA pseudouridine synthesis References: PMID:27268497 Sources: GOC:TermGenie, GO_REF:0000058 Relationships: is a type of positive regulation of RNA metabolic process [GO:0051254]; is_a GO:1905356; positively regulates snRNA pseudouridine synthesis [GO:0031120] Definition: Any process that activates or increases the frequency, rate or extent of snRNA pseudouridine synthesis.